{
  "gene_symbol": "CPA2",
  "gene_name": "Carboxypeptidase A2",
  "term_id": "GO:0005615",
  "term_label": "extracellular space",
  "gene": "UniProtKB:P48052"
}